{
  "gene_name": "Integral membrane protein GPR180",
  "term_id": "UNKNOWN:0002",
  "term_label": "Unknown biological process",
  "gene_symbol": "GPR180",
  "gene": "UniProtKB:Q86V85"
}